1,6-alpha-L-fucosidase activity [GO:0033938] (molecular function) Definition: Catalysis of the hydrolysis of (1->6) linkages between alpha-L-fucose and N-acetyl-D-glucosamine in glycopeptides such as immunoglobulin G glycopeptide and fucosyl-asialo-agalacto-fetuin. Also known as: 1,6-L-fucosyl-N-acetyl-D-glucosaminylglycopeptide fucohydrolase activity Relationships: is a type of alpha-L-fucosidase activity [GO:0004560] Sources: EC:3.2.1.127